{
  "gene_symbol": "FBN2",
  "gene_name": "Fibrillin-2",
  "gene": "UniProtKB:P35556",
  "term_id": "GO:0042593",
  "term_label": "glucose homeostasis"
}